{
  "term_label": "thiosulfate-cyanide sulfurtransferase activity",
  "term_id": "GO:0004792",
  "gene_name": "Adenylyltransferase and sulfurtransferase MOCS3",
  "gene": "UniProtKB:O95396",
  "gene_symbol": "MOCS3"
}